{
  "gene_symbol": "IRF5",
  "gene": "UniProtKB:Q13568",
  "term_label": "nucleus",
  "term_id": "GO:0005634",
  "gene_name": "Interferon regulatory factor 5"
}